fungal-type cell wall biogenesis [GO:0009272] (biological process) Sources: GOC:go_curators, GOC:mtg_sensu Regulation: regulated by GO:0032995 Definition: A cellular process that results in the biosynthesis of constituent macromolecules, assembly, and arrangement of constituent parts of a fungal-type cell wall. The fungal-type cell wall contains beta-glucan and may contain chitin. Relationships: is a type of cell wall biogenesis [GO:0042546]; is a type of fungal-type cell wall organization or biogenesis [GO:0071852] Subtypes: GO:0070591 Also known as: chitin- and beta-glucan-containing cell wall biogenesis, fungal-type cell wall anabolism, fungal-type cell wall biosynthetic process, fungal-type cell wall formation, fungal-type cell wall synthesis